{
  "term_label": "Z disc",
  "gene_name": "Alpha-actinin-1",
  "gene_symbol": "ACTN1",
  "gene": "UniProtKB:P12814",
  "term_id": "GO:0030018"
}